{
  "gene": "UniProtKB:Q5GH76",
  "term_id": "UNKNOWN:0001",
  "term_label": "Unknown molecular function",
  "gene_symbol": "XKR4",
  "gene_name": "XK-related protein 4"
}